type 5 metabotropic glutamate receptor binding [GO:0031802] (molecular function) Sources: GOC:mah, GOC:nln Also known as: type 5 metabotropic glutamate receptor ligand Definition: Binding to a type 5 metabotropic glutamate receptor. Relationships: is a type of G protein-coupled glutamate receptor binding [GO:0035256]